{
  "gene": "UniProtKB:Q5VTQ0",
  "gene_name": "Tetratricopeptide repeat protein 39B",
  "gene_symbol": "TTC39B",
  "term_id": "GO:0090181",
  "term_label": "regulation of cholesterol metabolic process"
}